{
  "gene_name": "Transmembrane protein 179",
  "term_label": "Unknown cellular component",
  "gene_symbol": "TMEM179",
  "term_id": "UNKNOWN:0003",
  "gene": "UniProtKB:Q6ZVK1"
}